{
  "term_label": "extracellular space",
  "gene_symbol": "MMP2",
  "gene": "UniProtKB:P08253",
  "gene_name": "72 kDa type IV collagenase",
  "term_id": "GO:0005615"
}